{
  "term_label": "Unknown biological process",
  "gene": "UniProtKB:Q8WWG1",
  "gene_name": "Pro-neuregulin-4, membrane-bound isoform",
  "term_id": "UNKNOWN:0002",
  "gene_symbol": "NRG4"
}